{
  "term_label": "positive regulation of cytosolic calcium ion concentration",
  "gene_name": "Atypical chemokine receptor 2",
  "term_id": "GO:0007204",
  "gene": "UniProtKB:O00590",
  "gene_symbol": "ACKR2"
}